{
  "gene_name": "Ferroxidase HEPHL1",
  "gene": "UniProtKB:Q6MZM0",
  "gene_symbol": "HEPHL1",
  "term_label": "ferroxidase activity",
  "term_id": "GO:0004322"
}